{
  "gene": "UniProtKB:Q9Y6W8",
  "term_label": "Unknown cellular component",
  "term_id": "UNKNOWN:0003",
  "gene_name": "Inducible T-cell costimulator",
  "gene_symbol": "ICOS"
}